{
  "term_id": "GO:0045892",
  "gene_name": "Zinc finger MYND domain-containing protein 15",
  "gene_symbol": "ZMYND15",
  "gene": "UniProtKB:Q9H091",
  "term_label": "negative regulation of DNA-templated transcription"
}